{
  "term_label": "nucleus",
  "gene": "UniProtKB:Q86V81",
  "gene_name": "THO complex subunit 4",
  "term_id": "GO:0005634",
  "gene_symbol": "ALYREF"
}